{
  "gene": "UniProtKB:P04049",
  "term_label": "MAP kinase kinase kinase activity",
  "gene_name": "RAF proto-oncogene serine_threonine-protein kinase",
  "gene_symbol": "RAF1",
  "term_id": "GO:0004709"
}